{
  "gene_name": "POTE ankyrin domain family member J",
  "gene_symbol": "POTEJ",
  "term_label": "actin filament",
  "term_id": "GO:0005884",
  "gene": "UniProtKB:P0CG39"
}